has part [BFO:0000051] (external)